regulation of lamellocyte differentiation [GO:0035203] (biological process) Definition: Any process that modulates the frequency, rate or extent of lamellocyte differentiation. Lamellocytes differentiate massively in the lymph glands after parasitization and are large flat cells devoted to encapsulation of invaders too large to be phagocytosed by plasmatocytes. Subtypes: negative regulation of lamellocyte differentiation [GO:0035204], positive regulation of lamellocyte differentiation [GO:0035205] Relationships: is a type of regulation of hemocyte differentiation [GO:0045610]; is a type of regulation of hemopoiesis [GO:1903706]; regulates lamellocyte differentiation [GO:0035171] References: PMID:14734104